{
  "term_label": "Unknown molecular function",
  "gene_name": "Paraneoplastic antigen Ma1",
  "term_id": "UNKNOWN:0001",
  "gene": "UniProtKB:Q8ND90",
  "gene_symbol": "PNMA1"
}